{
  "term_label": "negative regulation of cAMP/PKA signal transduction",
  "term_id": "GO:0141162",
  "gene": "UniProtKB:Q14123",
  "gene_symbol": "PDE1C",
  "gene_name": "Dual specificity calcium_calmodulin-dependent 3',5'-cyclic nucleotide phosphodiesterase 1C"
}